{
  "term_id": "GO:0042393",
  "term_label": "histone binding",
  "gene_symbol": "SSRP1",
  "gene_name": "FACT complex subunit SSRP1",
  "gene": "UniProtKB:Q08945"
}